{
  "term_label": "apoptotic signaling pathway",
  "gene": "UniProtKB:P08133",
  "gene_name": "Annexin A6",
  "term_id": "GO:0097190",
  "gene_symbol": "ANXA6"
}